{
  "gene": "UniProtKB:Q9HCE5",
  "gene_symbol": "METTL14",
  "term_label": "nucleus",
  "term_id": "GO:0005634",
  "gene_name": "N6-adenosine-methyltransferase non-catalytic subunit"
}